{
  "term_id": "UNKNOWN:0003",
  "term_label": "Unknown cellular component",
  "gene_symbol": "HAL",
  "gene": "UniProtKB:P42357",
  "gene_name": "Histidine ammonia-lyase"
}